{
  "term_id": "GO:0010494",
  "gene_symbol": "STAU2",
  "gene": "UniProtKB:Q9NUL3",
  "gene_name": "Double-stranded RNA-binding protein Staufen homolog 2",
  "term_label": "cytoplasmic stress granule"
}